{
  "gene": "UniProtKB:Q01101",
  "gene_name": "Insulinoma-associated protein 1",
  "term_label": "DNA-binding transcription repressor activity, RNA polymerase II-specific",
  "term_id": "GO:0001227",
  "gene_symbol": "INSM1"
}